{
  "term_id": "UNKNOWN:0002",
  "gene": "UniProtKB:Q9BYB4",
  "gene_symbol": "GNB1L",
  "term_label": "Unknown biological process",
  "gene_name": "Guanine nucleotide-binding protein subunit beta-like protein 1"
}